vascular associated smooth muscle cell fate determination [GO:0097083] (biological process) Definition: The process in which a cell becomes capable of differentiating autonomously into a vascular smooth muscle cell regardless of its environment; upon determination, the cell fate cannot be reversed. A vascular smooth muscle cell is a non-striated, elongated, spindle-shaped cell found lining the blood vessels. Sources: GOC:BHF Also known as: vascular smooth muscle cell fate determination Relationships: is a type of muscle cell fate determination [GO:0007521]; is part of vascular associated smooth muscle cell fate commitment [GO:0097081]